{
  "gene_symbol": "FABP5P3",
  "gene": "UniProtKB:A8MUU1",
  "gene_name": "Putative fatty acid-binding protein 5-like protein 3",
  "term_id": "GO:0005829",
  "term_label": "cytosol"
}